{
  "term_label": "negative regulation of MAPK cascade",
  "term_id": "GO:0043409",
  "gene_name": "Phosphatidylethanolamine-binding protein 1",
  "gene_symbol": "PEBP1",
  "gene": "UniProtKB:P30086"
}